{
  "gene_name": "Sushi domain-containing protein 6",
  "gene_symbol": "SUSD6",
  "term_label": "DNA damage response",
  "term_id": "GO:0006974",
  "gene": "UniProtKB:Q92537"
}